platelet-derived growth factor receptor signaling pathway [GO:0048008] (biological process) Subtypes: GO:0035790, platelet-derived growth factor receptor-beta signaling pathway [GO:0035791], GO:0038086 Definition: The series of molecular signals initiated by a ligand binding to a platelet-derived growth factor receptor on the surface of a target cell, and ending with the regulation of a downstream cellular process, e.g. transcription. Regulation: regulated by GO:0010640; positively regulated by positive regulation of platelet-derived growth factor receptor signaling pathway [GO:0010641]; negatively regulated by negative regulation of platelet-derived growth factor receptor signaling pathway [GO:0010642] Relationships: is a type of cell surface receptor protein tyrosine kinase signaling pathway [GO:0007169] Also known as: PDGF receptor signaling pathway, PDGF receptor signalling pathway, PDGFR signaling pathway Sources: GOC:ceb